{
  "term_label": "actin filament binding",
  "gene_symbol": "MPRIP",
  "gene_name": "Myosin phosphatase Rho-interacting protein",
  "gene": "UniProtKB:Q6WCQ1",
  "term_id": "GO:0051015"
}